{
  "term_label": "lysosome organization",
  "gene_name": "SNARE-associated protein Snapin",
  "term_id": "GO:0007040",
  "gene_symbol": "SNAPIN",
  "gene": "UniProtKB:O95295"
}